positive regulation of primary miRNA processing [GO:2000636] (biological process) Definition: Any process that activates or increases the frequency, rate or extent of primary microRNA processing. Relationships: is a type of positive regulation of miRNA processing [GO:1903800]; is a type of GO:2000634; positively regulates primary miRNA processing [GO:0031053] Also known as: positive regulation of pri-miRNA processing, positive regulation of primary microRNA processing Sources: GOC:dph, GOC:sl